{
  "gene": "UniProtKB:Q6S8J3",
  "gene_symbol": "POTEE",
  "gene_name": "POTE ankyrin domain family member E",
  "term_label": "actin filament",
  "term_id": "GO:0005884"
}